regulation of hydrogen peroxide-induced neuron intrinsic apoptotic signaling pathway [GO:1903383] (biological process) Definition: Any process that modulates the frequency, rate or extent of a hydrogen peroxide-induced neuron intrinsic apoptotic signaling pathway. Relationships: is a type of regulation of oxidative stress-induced neuron intrinsic apoptotic signaling pathway [GO:1903376]; is a type of regulation of intrinsic apoptotic signaling pathway in response to hydrogen peroxide [GO:1903750]; regulates neuron intrinsic apoptotic signaling pathway in response to hydrogen peroxide [GO:0036482] Subtypes: negative regulation of hydrogen peroxide-induced neuron intrinsic apoptotic signaling pathway [GO:1903384] Also known as: regulation of H2O2-induced neuron apoptosis, regulation of hydrogen peroxide-induced neuron apoptosis, regulation of hydrogen peroxide-induced neuronal apoptosis, regulation of H2O2-induced neuron intrinsic apoptotic signaling pathway, regulation of neuron intrinsic apoptotic signaling pathway in response to H2O2, regulation of neuron intrinsic apoptotic signaling pathway in response to hydrogen peroxide, regulation of neuron apoptosis in response to hydrogen peroxide Sources: GOC:PARL, GOC:TermGenie, GOC:bf, GO_REF:0000058